regulation of CD40 signaling pathway [GO:2000348] (biological process) Definition: Any process that modulates the frequency, rate or extent of signaling via the CD40 signaling pathway. Also known as: regulation of CD40 signalling pathway Subtypes: negative regulation of CD40 signaling pathway [GO:2000349], positive regulation of CD40 signaling pathway [GO:2000350] Sources: GOC:mah Relationships: is a type of GO:0009966; regulates CD40 signaling pathway [GO:0023035]